{
  "gene_name": "Metalloreductase STEAP3",
  "term_label": "endosome",
  "term_id": "GO:0005768",
  "gene": "UniProtKB:Q658P3",
  "gene_symbol": "STEAP3"
}